peptidoglycan catabolic process [GO:0009253] (biological process) References: PMID:9158729 Also known as: murein catabolic process, murein catabolism, peptidoglycan breakdown, peptidoglycan catabolism, peptidoglycan degradation Definition: The chemical reactions and pathways resulting in the breakdown of peptidoglycans, any of a class of glycoconjugates found in bacterial cell walls and consisting of long glycan strands of alternating residues of beta-(1,4) linked N-acetylglucosamine and N-acetylmuramic acid, cross-linked by short peptides. Relationships: is a type of peptidoglycan metabolic process [GO:0000270]; is a type of GO:0006027